cardiac vascular smooth muscle cell fate commitment [GO:0060949] (biological process) Subtypes: epicardium-derived cardiac vascular smooth muscle cell fate commitment [GO:0060985] Definition: The commitment of cells to a cardiac vascular smooth muscle cell fate and its capacity to differentiate into a cardiac vascular smooth muscle cell. Relationships: is a type of cardiac cell fate commitment [GO:0060911]; is a type of vascular associated smooth muscle cell fate commitment [GO:0097081]; is part of cardiac vascular smooth muscle cell differentiation [GO:0060947] Also known as: heart vascular smooth muscle cell fate commitment Sources: GOC:mtg_heart